{
  "term_label": "Unknown cellular component",
  "gene_symbol": "MMP3",
  "gene": "UniProtKB:P08254",
  "gene_name": "Stromelysin-1",
  "term_id": "UNKNOWN:0003"
}